vacuole fusion [GO:0097576] (biological process) Sources: GOC:pr, GOC:vw, Wikipedia:Vacuole Definition: Merging of two or more vacuoles, or of vacuoles and vesicles within a cell to form a single larger vacuole. Relationships: is a type of vacuole organization [GO:0007033]; is a type of GO:0048284 Subtypes: vacuole fusion, non-autophagic [GO:0042144], GO:0051469